Noc4p-Nop14p complex [GO:0030692] (cellular component) Definition: A heterodimer associated with precursors of the eukaryotic small ribosomal subunit, including the 90S preribosome; involved in small subunit biogenesis. Relationships: is a type of Noc complex [GO:0030689]; is part of GO:0030686; is part of GO:0030688 Note: Noc complexes exhibit a dynamic intranuclear location; consider also annotating to 'nucleolus ; GO:0005730' and/or 'nucleoplasm ; GO:0005654' and/or 'nuclear pore ; GO:0005643'. Note that the term name uses Saccharomyces gene product names because no other names have yet arisen for this complex; the term nevertheless can be used for analogous complexes in other eukaryotes, and the name can be changed if better wording is found. References: PMID:12446671 Also known as: Nop7 complex, Nop7 subcomplex